{
  "term_id": "GO:0000978",
  "gene": "UniProtKB:Q8TD94",
  "gene_name": "Krueppel-like factor 14",
  "term_label": "RNA polymerase II cis-regulatory region sequence-specific DNA binding",
  "gene_symbol": "KLF14"
}